{
  "gene_symbol": "TTF2",
  "term_label": "DNA repair",
  "term_id": "GO:0006281",
  "gene": "UniProtKB:Q9UNY4",
  "gene_name": "Transcription termination factor 2"
}